{
  "term_label": "microtubule bundle formation",
  "gene_symbol": "GAS2L1",
  "term_id": "GO:0001578",
  "gene": "UniProtKB:Q99501",
  "gene_name": "GAS2-like protein 1"
}